{
  "gene": "UniProtKB:Q13445",
  "term_id": "GO:0030134",
  "gene_name": "Transmembrane emp24 domain-containing protein 1",
  "gene_symbol": "TMED1",
  "term_label": "COPII-coated ER to Golgi transport vesicle"
}